methanol biosynthetic process [GO:0046169] (biological process) Relationships: is a type of GO:0015945; is a type of primary alcohol biosynthetic process [GO:0034309] Definition: The chemical reactions and pathways resulting in the formation of methanol, CH3-OH, a colorless, flammable, mobile, poisonous liquid, widely used as a solvent. Sources: GOC:ai Also known as: methanol anabolism, methanol biosynthesis, methanol formation, methanol synthesis